regulation of cellular response to alcohol [GO:1905957] (biological process) Subtypes: regulation of abscisic acid-activated signaling pathway [GO:0009787], GO:0120141, negative regulation of cellular response to alcohol [GO:1905958], positive regulation of cellular response to alcohol [GO:1905959] Definition: Any process that modulates the frequency, rate or extent of cellular response to alcohol. References: PMID:26434723 Sources: GOC:TermGenie, GO_REF:0000058 Relationships: is a type of regulation of cellular process [GO:0050794]; is a type of regulation of response to alcohol [GO:1901419]; regulates GO:0097306